{
  "gene_name": "Stromal interaction molecule 2",
  "term_label": "store-operated calcium entry",
  "term_id": "GO:0002115",
  "gene_symbol": "STIM2",
  "gene": "UniProtKB:Q9P246"
}